{
  "term_label": "sphingomyelin phosphodiesterase D activity",
  "gene_name": "Sphingomyelin phosphodiesterase 4",
  "term_id": "GO:0050290",
  "gene": "UniProtKB:Q9NXE4",
  "gene_symbol": "SMPD4"
}